{
  "term_id": "UNKNOWN:0002",
  "gene_name": "Nuclear pore complex protein Nup160",
  "gene_symbol": "NUP160",
  "gene": "UniProtKB:Q12769",
  "term_label": "Unknown biological process"
}